{
  "gene": "UniProtKB:Q96NU0",
  "term_id": "UNKNOWN:0001",
  "term_label": "Unknown molecular function",
  "gene_symbol": "CNTNAP3B",
  "gene_name": "Contactin-associated protein-like 3B"
}